{
  "gene_name": "Humanin-like 3",
  "gene_symbol": "MTRNR2L3",
  "term_id": "GO:0048019",
  "term_label": "receptor antagonist activity",
  "gene": "UniProtKB:P0CJ70"
}